{
  "gene_name": "Phosphatidate phosphatase LPIN3",
  "gene": "UniProtKB:Q9BQK8",
  "term_id": "GO:0045944",
  "gene_symbol": "LPIN3",
  "term_label": "positive regulation of transcription by RNA polymerase II"
}